{
  "gene_symbol": "YJU2B",
  "term_label": "U2-type spliceosomal complex",
  "gene": "UniProtKB:P13994",
  "term_id": "GO:0005684",
  "gene_name": "Probable splicing factor YJU2B"
}